regulation of endothelin production [GO:1904470] (biological process) References: PMID:15560120 Sources: GOC:TermGenie, GO_REF:0000058 Relationships: is a type of GO:0001817; regulates endothelin production [GO:1990775] Also known as: regulation of EDN1 secretion, regulation of EDN2 secretion, regulation of EDN3 secretion, regulation of endothelin secretion, regulation of endothelin-1 secretion, regulation of endothelin-2 secretion, regulation of endothelin-3 secretion Subtypes: GO:1904471, positive regulation of endothelin production [GO:1904472] Definition: Any process that modulates the frequency, rate or extent of endothelin production.